{
  "gene_symbol": "FZR1",
  "term_id": "GO:1990757",
  "term_label": "ubiquitin ligase activator activity",
  "gene_name": "Fizzy-related protein homolog",
  "gene": "UniProtKB:Q9UM11"
}